{
  "gene_name": "MAP kinase-activated protein kinase 3",
  "gene_symbol": "MAPKAPK3",
  "term_id": "GO:0034097",
  "gene": "UniProtKB:Q16644",
  "term_label": "response to cytokine"
}